{
  "term_label": "Unknown molecular function",
  "gene_name": "Immunoglobulin iota chain",
  "term_id": "UNKNOWN:0001",
  "gene": "UniProtKB:P12018",
  "gene_symbol": "VPREB1"
}